{
  "gene": "UniProtKB:Q92752",
  "gene_symbol": "TNR",
  "term_label": "extracellular matrix",
  "term_id": "GO:0031012",
  "gene_name": "Tenascin-R"
}